{
  "term_label": "prevention of polyspermy",
  "gene_symbol": "ASTL",
  "gene": "UniProtKB:Q6HA08",
  "gene_name": "Astacin-like metalloendopeptidase",
  "term_id": "GO:0060468"
}